{
  "gene_name": "Transient receptor potential cation channel subfamily M member 6",
  "gene": "UniProtKB:Q9BX84",
  "gene_symbol": "TRPM6",
  "term_id": "GO:0005262",
  "term_label": "calcium channel activity"
}